{
  "gene": "UniProtKB:Q9NR21",
  "term_label": "NAD+-protein mono-ADP-ribosyltransferase activity",
  "gene_symbol": "PARP11",
  "gene_name": "Protein mono-ADP-ribosyltransferase PARP11",
  "term_id": "GO:1990404"
}